{
  "term_label": "fusion of sperm to egg plasma membrane involved in single fertilization",
  "gene_symbol": "FREY1",
  "gene": "UniProtKB:C9JXX5",
  "term_id": "GO:0007342",
  "gene_name": "Protein Frey 1"
}